{
  "term_id": "GO:0035725",
  "gene_name": "Sodium_calcium exchanger 2",
  "term_label": "sodium ion transmembrane transport",
  "gene": "UniProtKB:Q9UPR5",
  "gene_symbol": "SLC8A2"
}